{
  "term_label": "perinuclear endoplasmic reticulum",
  "term_id": "GO:0097038",
  "gene_symbol": "OSBP2",
  "gene_name": "Oxysterol-binding protein 2",
  "gene": "UniProtKB:Q969R2"
}